presynaptic actin cytoskeleton organization [GO:0099140] (biological process) Definition: A process that is carried out at the cellular level which results in the assembly, arrangement of constituent parts, or disassembly of cytoskeletal structures comprising actin filaments and their associated proteins in the presynaptic actin cytoskeleton. Relationships: is a type of GO:0030036; is a type of GO:0099187 Sources: GOC:dos